{
  "gene_name": "Elongator complex protein 4",
  "gene": "UniProtKB:Q96EB1",
  "term_id": "UNKNOWN:0001",
  "gene_symbol": "ELP4",
  "term_label": "Unknown molecular function"
}